transaminase activity [GO:0008483] (molecular function) Also known as: aminotransferase activity Subtypes: GO:0003992, adenosylmethionine-8-amino-7-oxononanoate transaminase activity [GO:0004015], L-aspartate:2-oxoglutarate aminotransferase activity [GO:0004069], branched-chain-amino-acid transaminase activity [GO:0004084], GO:0004400, ornithine aminotransferase activity [GO:0004587], O-phospho-L-serine:2-oxoglutarate aminotransferase activity [GO:0004648], L-serine-pyruvate transaminase activity [GO:0004760], L-histidine:2-oxoglutarate aminotransferase activity [GO:0008110], GO:0008453, aromatic-amino-acid transaminase activity [GO:0008793], GO:0009016, valine-pyruvate transaminase activity [GO:0009042], GO:0010285, methionine-oxo-acid transaminase activity [GO:0010326], kynurenine-oxoglutarate transaminase activity [GO:0016212], beta-alanine:pyruvate transaminase activity [GO:0016223], 6-aminohexanoate transaminase activity [GO:0018719], diamine transaminase activity [GO:0019161], GO:0019162, pyridoxamine-phosphate transaminase activity [GO:0019163], GO:0019179, dTDP-4-amino-4,6-dideoxygalactose transaminase activity [GO:0019180], taurine-pyruvate aminotransferase activity [GO:0031299], putrescine--2-oxoglutarate transaminase activity [GO:0033094], thyroid-hormone transaminase activity [GO:0033852], aspartate-prephenate aminotransferase activity [GO:0033853], glutamate-prephenate aminotransferase activity [GO:0033854], GO:0033855, 4-aminobutyrate:2-oxoglutarate transaminase activity [GO:0034386], GO:0034387, GO:0043760, GO:0043825, D-lysine transaminase activity [GO:0043911], diaminobutyrate-2-oxoglutarate transaminase activity [GO:0045303], L-lysine 6-transaminase activity [GO:0045484], 4-amino-4-deoxychorismate synthase activity [GO:0046820], GO:0047297, GO:0047298, tryptophan-phenylpyruvate transaminase activity [GO:0047299], pyridoxamine-pyruvate transaminase activity [GO:0047300], valine-3-methyl-2-oxovalerate transaminase activity [GO:0047301], UDP-2-acetamido-4-amino-2,4,6-trideoxyglucose transaminase activity [GO:0047302], GO:0047303, GO:0047304, (R)-3-amino-2-methylpropionate-pyruvate transaminase activity [GO:0047305], D-methionine-pyruvate transaminase activity [GO:0047306], GO:0047307, alanine-oxomalonate transaminase activity [GO:0047308], dihydroxyphenylalanine transaminase activity [GO:0047309], GO:0047311, aromatic-amino-acid-glyoxylate transaminase activity [GO:0047313], kynurenine-glyoxylate transaminase activity [GO:0047315], GO:0047317, aspartate-phenylpyruvate transaminase activity [GO:0047319], D-4-hydroxyphenylglycine transaminase activity [GO:0047320], 2-aminoadipate transaminase activity [GO:0047536], 2-aminohexanoate transaminase activity [GO:0047537], 4-hydroxyglutamate transaminase activity [GO:0047578], GO:0047589, alanine-oxo-acid transaminase activity [GO:0047635], aminolevulinate transaminase activity [GO:0047665], GO:0047740, L-cysteine transaminase activity [GO:0047801], GO:0047802, D-alanine-2-oxoglutarate aminotransferase activity [GO:0047810], diiodotyrosine transaminase activity [GO:0047861], glycine:2-oxoglutarate aminotransferase activity [GO:0047958], lysine-pyruvate 6-transaminase activity [GO:0050065], methionine-glyoxylate transaminase activity [GO:0050094], GO:0050281, taurine-2-oxoglutarate transaminase activity [GO:0050322], L-lysine alpha-aminotransferase [GO:0062045], GO:0070529, L-glutamine aminotransferase activity [GO:0070548], UDP-4-amino-4-deoxy-L-arabinose aminotransferase [GO:0099620], GDP-4-dehydro-6-deoxy-D-mannose-4-aminotransferase activity [GO:0102933], 2-aminobutanoate transaminase activity [GO:0120554] Definition: Catalysis of the transfer of an amino group to an acceptor, usually a 2-oxo acid. Relationships: is a type of GO:0016769 Sources: EC:2.6.1.-